{
  "term_id": "GO:0015631",
  "gene_symbol": "TTLL1",
  "term_label": "tubulin binding",
  "gene": "UniProtKB:O95922",
  "gene_name": "Polyglutamylase complex subunit TTLL1"
}